{
  "gene_symbol": "EMID1",
  "term_id": "UNKNOWN:0001",
  "gene": "UniProtKB:Q96A84",
  "gene_name": "EMI domain-containing protein 1",
  "term_label": "Unknown molecular function"
}